immature B cell differentiation [GO:0002327] (biological process) Relationships: is a type of B cell differentiation [GO:0030183] Definition: The process in which a precursor cell type acquires the specialized features of an immature B cell. Also known as: immature B lymphocyte differentiation, immature B-cell differentiation, immature B-lymphocyte differentiation, immature B cell development Subtypes: pre-B cell differentiation [GO:0002329], transitional stage B cell differentiation [GO:0002332] Note: Note that immunologists typically use the word 'development' to refer to cells of B or T cell lineages undergoing the process that GO describes as 'cell differentiation'. References: PMID:16551251 Sources: GOC:jal, ISBN:0781735149